{
  "gene": "UniProtKB:A2VDF0",
  "gene_symbol": "FUOM",
  "gene_name": "Fucose mutarotase",
  "term_id": "UNKNOWN:0003",
  "term_label": "Unknown cellular component"
}